{
  "gene_name": "E3 ubiquitin-protein ligase RNF186",
  "gene": "UniProtKB:Q9NXI6",
  "term_id": "GO:0070534",
  "term_label": "protein K63-linked ubiquitination",
  "gene_symbol": "RNF186"
}